{
  "term_id": "GO:0005739",
  "gene_symbol": "COX7B2",
  "gene_name": "Cytochrome c oxidase subunit 7B2, mitochondrial",
  "term_label": "mitochondrion",
  "gene": "UniProtKB:Q8TF08"
}